{
  "gene_name": "Probable E3 ubiquitin-protein ligase HERC3",
  "gene_symbol": "HERC3",
  "gene": "UniProtKB:Q15034",
  "term_id": "GO:0006511",
  "term_label": "ubiquitin-dependent protein catabolic process"
}